spermatid nucleus differentiation [GO:0007289] (biological process) Sources: GOC:bf, GOC:dph, GOC:jl, GOC:mah Relationships: is a type of nucleus organization [GO:0006997]; is part of spermatid development [GO:0007286] Also known as: spermatid nuclear differentiation Definition: The specialization of the spermatid nucleus during the development of a spermatid into a mature male gamete competent for fertilization. Note: See also the Cell Ontology term 'spermatid ; CL:0000018'. Regulation: regulated by regulation of spermatid nuclear differentiation [GO:0045700]; negatively regulated by negative regulation of spermatid nuclear differentiation [GO:0045701]; positively regulated by positive regulation of spermatid nuclear differentiation [GO:0045702]